{
  "term_id": "UNKNOWN:0003",
  "gene_symbol": "EIPR1",
  "gene": "UniProtKB:Q53HC9",
  "term_label": "Unknown cellular component",
  "gene_name": "EARP and GARP complex-interacting protein 1"
}